{
  "term_id": "GO:0005737",
  "gene_name": "E3 ubiquitin-protein ligase TRIM69",
  "gene": "UniProtKB:Q86WT6",
  "term_label": "cytoplasm",
  "gene_symbol": "TRIM69"
}